corticosterone secretion [GO:0035934] (biological process) Sources: GOC:sl Regulation: regulated by regulation of corticosterone secretion [GO:2000852]; negatively regulated by negative regulation of corticosterone secretion [GO:2000853]; positively regulated by positive regulation of corticosterone secretion [GO:2000854] Relationships: is a type of organic hydroxy compound transport [GO:0015850]; is a type of glucocorticoid secretion [GO:0035933] Definition: The regulated release of corticosterone into the circulatory system. Corticosterone is a 21-carbon steroid hormone of the corticosteroid type produced in the cortex of the adrenal glands.